cell chemotaxis to fibroblast growth factor [GO:0035766] (biological process) Regulation: regulated by regulation of cell chemotaxis to fibroblast growth factor [GO:1904847]; negatively regulated by negative regulation of cell chemotaxis to fibroblast growth factor [GO:1904848]; positively regulated by positive regulation of cell chemotaxis to fibroblast growth factor [GO:1904849] Subtypes: endothelial cell chemotaxis to fibroblast growth factor [GO:0035768] Definition: The directed movement of a motile cell in response to the presence of fibroblast growth factor (FGF). Sources: GOC:BHF Relationships: is a type of GO:0060326; BFO_0000050 cellular response to fibroblast growth factor stimulus [GO:0044344]